{
  "term_label": "cytokine receptor activity",
  "gene_name": "Interferon gamma receptor 1",
  "term_id": "GO:0004896",
  "gene": "UniProtKB:P15260",
  "gene_symbol": "IFNGR1"
}